peptidyl-lysine dimethylation [GO:0018027] (biological process) Definition: The methylation of peptidyl-lysine to form peptidyl-N6,N6-dimethyl-L-lysine. Relationships: is a type of peptidyl-lysine methylation [GO:0018022] Sources: RESID:AA0075